{
  "term_id": "GO:0009897",
  "gene": "UniProtKB:P25024",
  "gene_name": "C-X-C chemokine receptor type 1",
  "term_label": "external side of plasma membrane",
  "gene_symbol": "CXCR1"
}